{
  "term_id": "GO:0005789",
  "gene_symbol": "TMEM170A",
  "gene": "UniProtKB:Q8WVE7",
  "gene_name": "Transmembrane protein 170A",
  "term_label": "endoplasmic reticulum membrane"
}